{
  "gene_symbol": "RTN2",
  "term_label": "neuron projection",
  "gene_name": "Reticulon-2",
  "term_id": "GO:0043005",
  "gene": "UniProtKB:O75298"
}